{
  "gene_symbol": "SHPK",
  "gene_name": "Sedoheptulokinase",
  "term_id": "GO:0071222",
  "gene": "UniProtKB:Q9UHJ6",
  "term_label": "cellular response to lipopolysaccharide"
}